{
  "gene_name": "Golgin subfamily A member 8R",
  "term_id": "GO:0032580",
  "term_label": "Golgi cisterna membrane",
  "gene": "UniProtKB:I6L899",
  "gene_symbol": "GOLGA8R"
}